G protein-coupled receptor homodimeric complex [GO:0038038] (cellular component) Definition: A protein complex that contains two G protein-coupled receptors (GPCRs) of the same subtype. Formation of a GPCR homodimer may be important for the transport of newly formed receptors to the cell surface, and the function of the receptor. Also known as: G-protein coupled receptor homodimer, G-protein coupled receptor homodimeric complex, GPCR homodimer References: PMID:10713101, PMID:16670762 Sources: GOC:al, GOC:bf Relationships: is a type of G protein-coupled receptor dimeric complex [GO:0038037]